sigma factor activity [GO:0016987] (molecular function) Sources: GOC:txnOH-2018 Relationships: is a type of DNA-binding transcription factor activity [GO:0003700]; is part of regulation of DNA-templated transcription initiation [GO:2000142]; has part core promoter sequence-specific DNA binding [GO:0001046]; has part RNA polymerase core enzyme binding [GO:0043175] Definition: Sigma factors act as the promoter specificity subunit of eubacterial and plant plastid multisubunit RNA polymerases, whose core subunit composition is often described as alpha(2)-beta-beta-prime. Although sigma does not bind DNA on its own, when combined with the core to form the holoenzyme, the sigma factor binds specifically to promoter elements. The sigma subunit is released once elongation begins. Also known as: DNA-dependent RNA polymerase promoter selection factor, core DNA-dependent RNA polymerase binding promoter specificity activity, sigma transcription factor, bacterial sigma factor activity, plastid sigma factor activity, promoter selection factor activity